{
  "term_id": "GO:0005737",
  "gene_symbol": "NECAB3",
  "gene_name": "N-terminal EF-hand calcium-binding protein 3",
  "term_label": "cytoplasm",
  "gene": "UniProtKB:Q96P71"
}